{
  "gene": "UniProtKB:Q7Z628",
  "term_label": "Unknown cellular component",
  "gene_name": "Neuroepithelial cell-transforming gene 1 protein",
  "term_id": "UNKNOWN:0003",
  "gene_symbol": "NET1"
}